{
  "gene_symbol": "USP54",
  "gene_name": "Inactive ubiquitin carboxyl-terminal hydrolase 54",
  "gene": "UniProtKB:Q70EL1",
  "term_label": "Unknown cellular component",
  "term_id": "UNKNOWN:0003"
}